insulin receptor substrate binding [GO:0043560] (molecular function) Definition: Binding to an insulin receptor substrate (IRS) protein, an adaptor protein that bind to the transphosphorylated insulin and insulin-like growth factor receptors, are themselves phosphorylated and in turn recruit SH2 domain-containing signaling molecules to form a productive signaling complex. References: PMID:12829233 Also known as: IRS [protein] binding, IRS binding, insulin receptor substrate [protein] binding Relationships: is a type of protein binding [GO:0005515]